regulation of intestinal cholesterol absorption [GO:0030300] (biological process) Relationships: is a type of regulation of intestinal lipid absorption [GO:1904729]; regulates intestinal cholesterol absorption [GO:0030299] Definition: Any process that modulates the frequency, rate or extent of absorption of cholesterol into the blood, and the exclusion of other sterols from absorption. References: PMID:11099417 Sources: GOC:mah Subtypes: negative regulation of intestinal cholesterol absorption [GO:0045796], positive regulation of intestinal cholesterol absorption [GO:0045797]